dendriole [GO:0044293] (cellular component) References: PMID:8300904 Sources: GOC:jl, NIF_Subcellular:sao28175134, NIF_Subcellular:sao295057932 Definition: Small dendrites that makes up a brush structure found as the terminal specialization of a dendrite of a unipolar brush cell (UBC). Relationships: is a type of dendrite terminus [GO:0044292]